{
  "gene_symbol": "CHRNA1",
  "term_label": "acetylcholine receptor activity",
  "gene_name": "Acetylcholine receptor subunit alpha",
  "gene": "UniProtKB:P02708",
  "term_id": "GO:0015464"
}